nicotinate metabolic process [GO:1901847] (biological process) Subtypes: nicotinate catabolic process [GO:1901848], GO:1901849 Relationships: is a type of GO:0009820; is a type of monocarboxylic acid metabolic process [GO:0032787]; is a type of GO:0072524 Also known as: nicotinate metabolism Definition: The chemical reactions and pathways involving nicotinate. Sources: GOC:TermGenie, GOC:yaf, UniPathway:UPA00830